negative regulation of Schwann cell proliferation involved in axon regeneration [GO:1905045] (biological process) Also known as: down regulation of Schwann cell proliferation involved in axon regeneration, down-regulation of Schwann cell proliferation involved in axon regeneration, downregulation of Schwann cell proliferation involved in axon regeneration, inhibition of Schwann cell proliferation involved in axon regeneration Relationships: is a type of negative regulation of Schwann cell proliferation [GO:0010626]; is a type of GO:1905044; negatively regulates Schwann cell proliferation involved in axon regeneration [GO:0014011] References: PMID:22393241 Sources: GOC:BHF, GOC:BHF_miRNA, GOC:TermGenie, GOC:rph, GO_REF:0000058 Definition: Any process that stops, prevents or reduces the frequency, rate or extent of Schwann cell proliferation involved in axon regeneration.